erythrophore differentiation [GO:0048773] (biological process) Regulation: regulated by regulation of erythrophore differentiation [GO:0048778]; negatively regulated by GO:0048779; positively regulated by positive regulation of erythrophore differentiation [GO:0048780] Relationships: is a type of pigment cell differentiation [GO:0050931] Definition: The process in which a relatively unspecialized cell acquires the specialized features of an erythrophore cell. Erythrophores are pigment cells derived from the neural crest. They contain pteridine and/or carotenoid pigments in structures called pterinosomes or erythrosomes. This gives them an orange to red appearance. Also known as: erythrophore cell differentiation Sources: GOC:jid, GOC:mh